rixosome complex [GO:0120330] (cellular component) References: PMID:32491985, PMID:35355014 Sources: GOC:vw Relationships: is a type of GO:1902555 Also known as: rix1 complex Definition: A conserved RNA endonuclease complex required for spreading and epigenetic inheritance of heterochromatin. The rixosome contains six unique subunits: three structural subunits (Crb3, Rix1, and Ipi1) which form the core of the complex, and three catalytic subunits (the endonuclease Las1, the polynucleotide kinase Grc3, and the AAA-type ATPase Mdn1), which are involved in the processing of ribosomal RNA precursors. All subunits are essential for viability and are conserved from yeast to mammals, including humans.